{
  "gene_symbol": "KXD1",
  "gene_name": "KxDL motif-containing protein 1",
  "term_id": "GO:0099078",
  "gene": "UniProtKB:Q9BQD3",
  "term_label": "BORC complex"
}